{
  "term_label": "signal transduction",
  "term_id": "GO:0007165",
  "gene_name": "5'-AMP-activated protein kinase subunit beta-1",
  "gene": "UniProtKB:Q9Y478",
  "gene_symbol": "PRKAB1"
}